{
  "term_id": "GO:0005886",
  "gene": "UniProtKB:O75023",
  "term_label": "plasma membrane",
  "gene_symbol": "LILRB5",
  "gene_name": "Leukocyte immunoglobulin-like receptor subfamily B member 5"
}